learning or memory [GO:0007611] (biological process) References: PMID:8938125 Sources: GOC:jid Relationships: is a type of GO:0007610; is a type of cognition [GO:0050890] Definition: The acquisition and processing of information and/or the storage and retrieval of this information over time. Subtypes: learning [GO:0007612], GO:0007613, learned vocalization behavior or vocal learning [GO:0098598]